{
  "gene_symbol": "MRPL40",
  "term_label": "Unknown biological process",
  "term_id": "UNKNOWN:0002",
  "gene_name": "Large ribosomal subunit protein mL40",
  "gene": "UniProtKB:Q9NQ50"
}